endocannabinoid signaling pathway [GO:0071926] (BP) Definition: The series of molecular signals generated as a consequence of an endocannabinoid binding to a cell surface receptor. The pathway proceeds with the receptor transmitting the signal to a heterotrimeric G-protein complex and ends with regulation of a downstream cellular process, e.g. transcription. Endocannabinoids are small molecules derived from arachidonic acid, anandamide (arachidonoylethanolamide) and 2-arachidonoylglycerol. References: PMID:15550444 Sources: GOC:bf, GOC:mah Also known as: endocannabinoid signalling pathway Relationships: is a type of cannabinoid signaling pathway [GO:0038171] Subtypes: endocannabinoid signaling pathway involved in trans-synaptic signaling [GO:1905129] Regulation: regulated by regulation of endocannabinoid signaling pathway [GO:2000124]